{
  "term_label": "Unknown molecular function",
  "term_id": "UNKNOWN:0001",
  "gene_symbol": "TP53TG5",
  "gene_name": "TP53-target gene 5 protein",
  "gene": "UniProtKB:Q9Y2B4"
}